{
  "gene_name": "Sodium_potassium-transporting ATPase subunit beta-1-interacting protein 4",
  "term_label": "regulation of sodium ion transport",
  "gene": "UniProtKB:Q8IVV8",
  "term_id": "GO:0002028",
  "gene_symbol": "NKAIN4"
}